{
  "gene_symbol": "DNMT3A",
  "term_label": "DNA (cytosine-5-)-methyltransferase activity",
  "term_id": "GO:0003886",
  "gene": "UniProtKB:Q9Y6K1",
  "gene_name": "DNA (cytosine-5)-methyltransferase 3A"
}